{
  "gene_symbol": "KPNA5",
  "term_label": "nucleus",
  "term_id": "GO:0005634",
  "gene_name": "Importin subunit alpha-6",
  "gene": "UniProtKB:O15131"
}